{
  "term_label": "negative regulation of single stranded viral RNA replication via double stranded DNA intermediate",
  "gene_name": "DNA dC-dU-editing enzyme APOBEC-3C",
  "term_id": "GO:0045869",
  "gene": "UniProtKB:Q9NRW3",
  "gene_symbol": "APOBEC3C"
}